{
  "gene_name": "Protein FAM193B",
  "term_label": "Unknown molecular function",
  "gene": "UniProtKB:Q96PV7",
  "gene_symbol": "FAM193B",
  "term_id": "UNKNOWN:0001"
}